{
  "term_label": "nuclear migration",
  "gene": "UniProtKB:O95359",
  "gene_name": "Transforming acidic coiled-coil-containing protein 2",
  "term_id": "GO:0007097",
  "gene_symbol": "TACC2"
}